positive regulation of muscle filament sliding [GO:1904114] (biological process) Also known as: up regulation of muscle filament sliding, up-regulation of muscle filament sliding, upregulation of muscle filament sliding, activation of muscle filament sliding References: PMID:25717181 Sources: GOC:TermGenie, GOC:kmv, GO_REF:0000058 Relationships: is a type of GO:0032971; is a type of GO:1903116; positively regulates muscle filament sliding [GO:0030049] Definition: Any process that activates or increases the frequency, rate or extent of muscle filament sliding.